{
  "term_label": "Unknown cellular component",
  "gene_symbol": "PYROXD1",
  "gene": "UniProtKB:Q8WU10",
  "gene_name": "Pyridine nucleotide-disulfide oxidoreductase domain-containing protein 1",
  "term_id": "UNKNOWN:0003"
}